{
  "term_label": "cytosol",
  "term_id": "GO:0005829",
  "gene_name": "Casein kinase II subunit alpha",
  "gene": "UniProtKB:P68400",
  "gene_symbol": "CSNK2A1"
}